neutrophil-mediated killing of fungus [GO:0070947] (BP) Definition: The directed killing of a fungal cell by a neutrophil. Relationships: is a type of neutrophil-mediated killing of symbiont cell [GO:0070943]; is part of defense response to fungus [GO:0050832] Regulation: regulated by regulation of neutrophil mediated killing of fungus [GO:0070953]; negatively regulated by negative regulation of neutrophil mediated killing of fungus [GO:0070959]; positively regulated by GO:0070965 Sources: GOC:add, ISBN:0781765196 Also known as: neutrophil mediated killing of fungus